{
  "term_label": "extracellular matrix organization",
  "gene_symbol": "ADAMTS12",
  "term_id": "GO:0030198",
  "gene": "UniProtKB:P58397",
  "gene_name": "A disintegrin and metalloproteinase with thrombospondin motifs 12"
}